{
  "term_id": "GO:0005763",
  "term_label": "mitochondrial small ribosomal subunit",
  "gene_name": "Small ribosomal subunit protein uS7m",
  "gene_symbol": "MRPS7",
  "gene": "UniProtKB:Q9Y2R9"
}